slime layer organization [GO:0045231] (biological process) Also known as: slime layer organisation, slime layer organization and biogenesis Sources: GOC:ai Definition: A process that is carried out at the cellular level which results in the assembly, arrangement of constituent parts, or disassembly of a slime layer. A slime layer is an easily removed, diffuse, unorganized layer of extracellular material that surrounds a cell. Subtypes: GO:0045228 Relationships: is a type of GO:0045229